intracellular lysine homeostasis [GO:0090463] (biological process) Definition: A homeostatic process involved in the maintenance of a steady state level of lysine within a cell. Sources: GOC:tb Relationships: is a type of intracellular amino acid homeostasis [GO:0080144] Also known as: cellular lysine homeostasis, lysine homeostasis